{
  "gene": "UniProtKB:Q5T2N8",
  "term_label": "Unknown molecular function",
  "gene_name": "ATPase family AAA domain-containing protein 3C",
  "gene_symbol": "ATAD3C",
  "term_id": "UNKNOWN:0001"
}